(+)-delta-cadinene synthase activity [GO:0047461] (molecular function) Relationships: is a type of sesquiterpene synthase activity [GO:0010334] Definition: Catalysis of the reaction: 2-trans,6-trans-farnesyl diphosphate = diphosphate + (+)-delta-cadinene. Sources: EC:4.2.3.13, MetaCyc:4.6.1.11-RXN Also known as: 2-trans,6-trans-farnesyl-diphosphate diphosphate-lyase (cyclizing, (+)-delta-cadinene-forming), D-cadinene synthase activity